negative regulation of mitotic chromosome condensation [GO:1905213] (biological process) Definition: Any process that stops, prevents or reduces the frequency, rate or extent of mitotic chromosome condensation. Relationships: is a type of negative regulation of cell cycle process [GO:0010948]; is a type of negative regulation of chromosome condensation [GO:1902340]; is a type of regulation of mitotic chromosome condensation [GO:1903379]; negatively regulates GO:0007076 References: PMID:23219725 Sources: GOC:TermGenie, GO_REF:0000058